gap junction-mediated intercellular transport [GO:1990349] (biological process) Relationships: is a type of intercellular transport [GO:0010496] References: PMID:14506308, PMID:23261543 Sources: GOC:hjd, Wikipedia:Gap_junction Definition: The movement of substances between cells via gap junctions. A gap junction is a fine cytoplasmic channel, found in animal cells, that connects the cytoplasm of one cell to that of an adjacent cell, allowing ions and other molecules to pass freely between the two cells.